{
  "term_label": "protein kinase binding",
  "term_id": "GO:0019901",
  "gene_symbol": "SPDYE3",
  "gene_name": "Speedy protein E3",
  "gene": "UniProtKB:A6NKU9"
}